involution involved in gastrulation with mouth forming second [GO:0055110] (biological process) Definition: The inturning of an epithelial sheet over the basal surface of an outer layer involved in deuterostomic gastrulation. Sources: ISBN:0878932437 Relationships: is a type of embryonic morphogenesis [GO:0048598]; is a type of morphogenesis of an epithelial fold [GO:0060571]; is part of gastrulation with mouth forming second [GO:0001702]